{
  "term_label": "neuron projection",
  "gene_symbol": "OPRD1",
  "gene": "UniProtKB:P41143",
  "gene_name": "Delta-type opioid receptor",
  "term_id": "GO:0043005"
}